{
  "gene_symbol": "BBS9",
  "gene": "UniProtKB:Q3SYG4",
  "term_label": "BBSome",
  "term_id": "GO:0034464",
  "gene_name": "Protein PTHB1"
}